{
  "term_id": "GO:0034045",
  "gene_name": "Ubiquitin-like protein ATG12",
  "gene": "UniProtKB:O94817",
  "gene_symbol": "ATG12",
  "term_label": "phagophore assembly site membrane"
}